{
  "term_label": "Unknown molecular function",
  "term_id": "UNKNOWN:0001",
  "gene_symbol": "CWC27",
  "gene": "UniProtKB:Q6UX04",
  "gene_name": "Spliceosome-associated protein CWC27 homolog"
}